TRAIL death-inducing signaling complex [GO:0031266] (CC) Relationships: is a type of death-inducing signaling complex [GO:0031264] References: PMID:12628743, PMID:12655293 Definition: A protein complex formed upon binding of TRAIL to its ligand. The complex includes FADD/Mort1 and procaspase-8 addition to the ligand-bound receptor. Also known as: TRAIL DISC, TRAIL death-inducing signalling complex